{
  "gene_name": "Proline and serine-rich protein 3",
  "term_label": "Unknown biological process",
  "term_id": "UNKNOWN:0002",
  "gene_symbol": "PROSER3",
  "gene": "UniProtKB:Q2NL68"
}